peptidyl-aspartic acid 3-dioxygenase activity [GO:0062101] (molecular function) References: PMID:1378441, PMID:1856229 Sources: RHEA:11508 Relationships: is a type of 2-oxoglutarate-dependent dioxygenase activity [GO:0016706]; is a type of catalytic activity, acting on a protein [GO:0140096] Also known as: peptide-aspartate beta-dioxygenase activity, aspartate beta-hydroxylase activity, aspartyl/asparaginyl beta-hydroxylase activity, aspartylpeptide beta-dioxygenase activity, peptide-L-aspartate,2-oxoglutarate:oxygen oxidoreductase (3-hydroxylating) activity Definition: Catalysis of the reaction: protein L-aspartate + 2-oxoglutarate + O2 = protein 3-hydroxy-L-aspartate + succinate + CO2.